{
  "gene_name": "Leucine zipper putative tumor suppressor 3",
  "term_id": "GO:0061001",
  "gene_symbol": "LZTS3",
  "gene": "UniProtKB:O60299",
  "term_label": "regulation of dendritic spine morphogenesis"
}